{
  "gene": "UniProtKB:Q92806",
  "gene_name": "G protein-activated inward rectifier potassium channel 3",
  "term_label": "inward rectifier potassium channel activity",
  "gene_symbol": "KCNJ9",
  "term_id": "GO:0005242"
}